{
  "gene": "UniProtKB:Q9NSC5",
  "term_id": "GO:2001256",
  "gene_symbol": "HOMER3",
  "gene_name": "Homer protein homolog 3",
  "term_label": "regulation of store-operated calcium entry"
}